glycerophospholipid biosynthetic process [GO:0046474] (biological process) Definition: The chemical reactions and pathways resulting in the formation of glycerophospholipids, any derivative of glycerophosphate that contains at least one O-acyl, O-alkyl, or O-alkenyl group attached to the glycerol residue. Sources: ISBN:0198506732 Also known as: glycerophospholipid anabolism, glycerophospholipid biosynthesis, glycerophospholipid formation, glycerophospholipid synthesis, phosphoglyceride biosynthesis, phosphoglyceride biosynthetic process Subtypes: phosphatidylethanolamine biosynthetic process [GO:0006646], phosphatidic acid biosynthetic process [GO:0006654], phosphatidylglycerol biosynthetic process [GO:0006655], phosphatidylcholine biosynthetic process [GO:0006656], phosphatidylserine biosynthetic process [GO:0006659], phosphatidylinositol biosynthetic process [GO:0006661], GO:0006663, CDP-diacylglycerol biosynthetic process [GO:0016024], lysobisphosphatidic acid biosynthetic process [GO:2001312] Relationships: is a type of glycerophospholipid metabolic process [GO:0006650]; is a type of phospholipid biosynthetic process [GO:0008654]; is a type of glycerolipid biosynthetic process [GO:0045017]